{
  "gene": "UniProtKB:Q969H4",
  "gene_symbol": "CNKSR1",
  "gene_name": "Connector enhancer of kinase suppressor of ras 1",
  "term_label": "protein-macromolecule adaptor activity",
  "term_id": "GO:0030674"
}